{
  "gene_symbol": "FRS2",
  "gene_name": "Fibroblast growth factor receptor substrate 2",
  "gene": "UniProtKB:Q8WU20",
  "term_label": "cell-cell junction",
  "term_id": "GO:0005911"
}